pyridoxal 4-dehydrogenase activity [GO:0050235] (molecular function) Sources: EC:1.1.1.107, RHEA:21336 Relationships: is a type of oxidoreductase activity, acting on the CH-OH group of donors, NAD or NADP as acceptor [GO:0016616] Also known as: pyridoxal dehydrogenase activity, pyridoxal:NAD+ 4-oxidoreductase activity Definition: Catalysis of the reaction: NAD+ + pyridoxal = 4-pyridoxolactone + H+ + NADH.